structural constituent of cytoskeleton [GO:0005200] (molecular function) Sources: GOC:mah Relationships: is a type of structural molecule activity [GO:0005198]; is part of cytoskeleton organization [GO:0007010]; occurs in cytoskeleton [GO:0005856] Subtypes: GO:0098699, structural constituent of postsynaptic actin cytoskeleton [GO:0098973], GO:0099184 Definition: The action of a molecule that contributes to the structural integrity of a cytoskeletal structure.